{
  "term_id": "GO:0017136",
  "term_label": "histone deacetylase activity, NAD-dependent",
  "gene_symbol": "SIRT2",
  "gene": "UniProtKB:Q8IXJ6",
  "gene_name": "NAD-dependent protein deacetylase sirtuin-2"
}